{
  "gene": "UniProtKB:P62312",
  "term_id": "GO:0000932",
  "gene_symbol": "LSM6",
  "gene_name": "U6 snRNA-associated Sm-like protein LSm6",
  "term_label": "P-body"
}